circadian temperature homeostasis [GO:0060086] (BP) Sources: GOC:dph, GOC:tb Definition: Any homeostatic process in which an organism modulates its internal body temperature at different values with a regularity of approximately 24 hours. Relationships: is a type of temperature homeostasis [GO:0001659]; is a type of circadian rhythm [GO:0007623] Also known as: circadian thermoregulation, circadian regulation of body temperature